{
  "gene": "UniProtKB:Q8NC26",
  "gene_name": "Zinc finger protein 114",
  "term_label": "regulation of DNA-templated transcription",
  "term_id": "GO:0006355",
  "gene_symbol": "ZNF114"
}